{
  "term_id": "GO:0005737",
  "gene": "UniProtKB:Q5F1R6",
  "gene_name": "DnaJ homolog subfamily C member 21",
  "term_label": "cytoplasm",
  "gene_symbol": "DNAJC21"
}